{
  "term_id": "GO:0000070",
  "gene": "UniProtKB:Q86Y91",
  "gene_symbol": "KIF18B",
  "gene_name": "Kinesin-like protein KIF18B",
  "term_label": "mitotic sister chromatid segregation"
}